{
  "term_id": "GO:0036126",
  "gene": "UniProtKB:Q8NA56",
  "gene_symbol": "TTC29",
  "term_label": "sperm flagellum",
  "gene_name": "Tetratricopeptide repeat protein 29"
}